{
  "gene_symbol": "ETDB",
  "gene": "UniProtKB:P0DPP9",
  "term_label": "Unknown molecular function",
  "gene_name": "Embryonic testis differentiation protein homolog B",
  "term_id": "UNKNOWN:0001"
}